response to anesthetic [GO:0072347] (biological process) Definition: Any process that results in a change in state or activity of a cell or an organism (in terms of movement, secretion, enzyme production, gene expression, etc.) as a result of an anesthetic stimulus. An anesthetic is a substance that causes loss of feeling, awareness, or sensation. Also known as: response to anaesthetic Sources: GOC:sart Relationships: is a type of response to chemical [GO:0042221]